maintenance of viral latency [GO:0019044] (biological process) Also known as: latent virus maintenance, prophage maintenance, provirus maintenance Relationships: is a type of viral process [GO:0016032]; BFO_0000050 GO:0019042 Definition: The perpetuation of a latent state, generally by repressing the viruses own lytic genes expression and ensuring expression of viral genes which function to keep the viral genome from being detected by the host defense mechanisms. Sources: GOC:jl